{
  "term_id": "GO:0004861",
  "gene_symbol": "CDKN2D",
  "gene_name": "Cyclin-dependent kinase 4 inhibitor D",
  "term_label": "cyclin-dependent protein serine/threonine kinase inhibitor activity",
  "gene": "UniProtKB:P55273"
}